{
  "gene_name": "Cyclin-dependent kinase 8",
  "term_id": "UNKNOWN:0002",
  "gene_symbol": "CDK8",
  "gene": "UniProtKB:P49336",
  "term_label": "Unknown biological process"
}